phosphatidylserine exposure on apoptotic cell surface [GO:0070782] (biological process) Regulation: regulated by regulation of phosphatidylserine exposure on apoptotic cell surface [GO:1905780]; negatively regulated by GO:1905781; positively regulated by positive regulation of phosphatidylserine exposure on apoptotic cell surface [GO:1905782] Also known as: externalization of phosphatidylserine References: PMID:11536005 Sources: GOC:mah, GOC:mtg_apoptosis, GOC:rk Note: In normal cells, phosphatidylserine residues are found exclusively on the inner side of the cellular membrane. During apoptosis, phosphatidylserine is transported to the outer cell surface by scramblase proteins. This event acts as an "eat-me" signal for macrophages to dispose of the dying cell. When annotating to this term, curators should be aware of the following: 1) phosphatidylserine exposure on the cell surface can occur in circumstances other than apoptosis (for example, when blood platelets are activated, they expose phosphatidylserine to trigger the clotting system, see PMID:21107324). Do not annotate to GO:0070782 unless phosphatidylserine exposure is shown to be part of an apoptotic event. 2) Caution should be applied when a study quotes annexin V assays. The annexin A5 protein binds to phosphatidylserine-containing membrane surfaces, which are usually only present on the inner leaflet of the membrane. However, in cells undergoing apoptosis, phosphatidylserine becomes exposed on the outer leaflet of the membrane. A positive annexin assay can therefore be linked to apoptotic death, but it shouldn't be confused with molecular events strictly involved in the process of phosphatidylserine exposure. Definition: A phospholipid scrambling process that results in the appearance of phosphatidylserine on the outer leaflet of the plasma membrane of an apoptotic cell, which acts as an 'eat-me' signal for engulfing cells. Phosphatidylserine is exposed on the apoptotic cell surface by a phospholipid scramblase activity. Relationships: is a type of plasma membrane phospholipid scrambling [GO:0017121]; is part of execution phase of apoptosis [GO:0097194]; has part GO:0017128